{
  "gene": "UniProtKB:Q14541",
  "term_label": "RNA polymerase II cis-regulatory region sequence-specific DNA binding",
  "gene_symbol": "HNF4G",
  "gene_name": "Hepatocyte nuclear factor 4-gamma",
  "term_id": "GO:0000978"
}